{
  "term_label": "extracellular space",
  "gene_name": "Growth_differentiation factor 11",
  "term_id": "GO:0005615",
  "gene": "UniProtKB:O95390",
  "gene_symbol": "GDF11"
}